{
  "term_label": "plasma membrane",
  "gene_name": "Olfactory receptor 10G7",
  "term_id": "GO:0005886",
  "gene": "UniProtKB:Q8NGN6",
  "gene_symbol": "OR10G7"
}